glycerol-3-phosphate dehydrogenase (quinone) activity [GO:0004368] (molecular function) Definition: Catalysis of the reaction: sn-glycerol 3-phosphate + a quinone = glycerone phosphate + a quinol. Sources: EC:1.1.5.3 Also known as: FAD-dependent glycerol-3-phosphate dehydrogenase, L-glycerophosphate dehydrogenase activity, flavin-linked glycerol-3-phosphate dehydrogenase, glycerol-3-phosphate CoQ reductase, glycerophosphate dehydrogenase activity, sn-glycerol-3-phosphate dehydrogenase activity Relationships: is a type of oxidoreductase activity, acting on the CH-OH group of donors, quinone or similar compound as acceptor [GO:0016901]